{
  "term_id": "GO:1904825",
  "gene_name": "GAS2-like protein 1",
  "gene_symbol": "GAS2L1",
  "gene": "UniProtKB:Q99501",
  "term_label": "protein localization to microtubule plus-end"
}